{
  "gene_symbol": "ZNF630",
  "gene": "UniProtKB:Q2M218",
  "term_id": "GO:0006357",
  "term_label": "regulation of transcription by RNA polymerase II",
  "gene_name": "Zinc finger protein 630"
}